positive regulation of calcium ion export across plasma membrane [GO:1905914] (biological process) References: PMID:22362515 Sources: GOC:BHF, GOC:BHF_miRNA, GOC:TermGenie, GOC:rph, GO_REF:0000058 Also known as: positive regulation of calcium ion efflux from cell, positive regulation of calcium ion export from cell, up regulation of calcium ion efflux from cell, up regulation of calcium ion export from cell, up-regulation of calcium ion efflux from cell, up-regulation of calcium ion export from cell, upregulation of calcium ion efflux from cell, upregulation of calcium ion export from cell, activation of calcium ion efflux from cell, activation of calcium ion export from cell Relationships: is a type of positive regulation of calcium ion transmembrane transport [GO:1904427]; is a type of regulation of calcium ion export across plasma membrane [GO:1905912]; positively regulates GO:1990034 Definition: Any process that activates or increases the frequency, rate or extent of calcium ion export across the plasma membrane.